{
  "gene_name": "Mothers against decapentaplegic homolog 4",
  "gene_symbol": "SMAD4",
  "term_id": "GO:0030509",
  "term_label": "BMP signaling pathway",
  "gene": "UniProtKB:Q13485"
}